{
  "term_id": "GO:0004565",
  "gene": "UniProtKB:Q9H227",
  "gene_symbol": "GBA3",
  "gene_name": "Cytosolic beta-glucosidase",
  "term_label": "beta-galactosidase activity"
}